Langerhans cell differentiation [GO:0061520] (biological process) References: PMID:22729249 Sources: GOC:dph Definition: The process in which a precursor cell type acquires the specialized features of a Langerhans cell. Relationships: is_a myeloid dendritic cell differentiation [GO:0043011]